colanic acid biosynthetic process [GO:0009242] (biological process) Relationships: is a type of macromolecule biosynthetic process [GO:0009059]; is a type of colanic acid metabolic process [GO:0046377]; is a type of carbohydrate derivative biosynthetic process [GO:1901137] Sources: GOC:ai Also known as: M antigen biosynthesis, M antigen biosynthetic process, colanic acid anabolism, colanic acid biosynthesis, colanic acid formation, colanic acid synthesis Definition: The chemical reactions and pathways resulting in the formation of colanic acid, a capsular bacterial polysaccharide.